{
  "term_label": "trace-amine receptor activity",
  "term_id": "GO:0001594",
  "gene_symbol": "TAAR6",
  "gene_name": "Trace amine-associated receptor 6",
  "gene": "UniProtKB:Q96RI8"
}